{
  "gene_name": "RNA-binding protein 42",
  "gene_symbol": "RBM42",
  "term_label": "Unknown biological process",
  "gene": "UniProtKB:Q9BTD8",
  "term_id": "UNKNOWN:0002"
}